{
  "term_id": "GO:0008296",
  "gene_name": "Three-prime repair exonuclease 1",
  "term_label": "3'-5'-DNA exonuclease activity",
  "gene_symbol": "TREX1",
  "gene": "UniProtKB:Q9NSU2"
}